detection of muscle inactivity involved in regulation of muscle adaptation [GO:0014884] (BP) Relationships: is a type of GO:0014869; is a type of response to muscle inactivity involved in regulation of muscle adaptation [GO:0014877] Definition: The series of events in which a muscle inactivity stimulus is received by a cell and converted into a molecular signal. This occurs as part of the regulation of muscle adaptation. Sources: GOC:ef, GOC:mtg_muscle